trabecular meshwork development [GO:0002930] (BP) References: PMID:20568247 Relationships: is a type of tissue development [GO:0009888]; is part of camera-type eye development [GO:0043010] Definition: The progression of the trabecular meshwork over time, from its formation to the mature structure. The trabecular meshwork is a fenestrated endothelial-like tissue situated at the intersection of the cornea and the iris. The trabecular meshwork provides drainage for the aqueous humor.